thymidine catabolic process [GO:0006214] (biological process) Definition: The chemical reactions and pathways resulting in the breakdown of thymidine, deoxyribosylthymine thymine 2-deoxyriboside, a deoxynucleoside very widely distributed but occurring almost entirely as phosphoric esters in deoxynucleotides and deoxyribonucleic acid, DNA. Relationships: is a type of GO:0046104; is a type of pyrimidine deoxyribonucleoside catabolic process [GO:0046127] Sources: GOC:go_curators Also known as: deoxyribosylthymine catabolic process, deoxyribosylthymine catabolism, thymidine breakdown, thymidine catabolism, thymidine degradation